{
  "gene_name": "Excitatory amino acid transporter 4",
  "term_label": "glutamate:sodium symporter activity",
  "gene_symbol": "SLC1A6",
  "gene": "UniProtKB:P48664",
  "term_id": "GO:0015501"
}